{
  "term_label": "cytoplasm",
  "gene_symbol": "AGO4",
  "gene": "UniProtKB:Q9HCK5",
  "term_id": "GO:0005737",
  "gene_name": "Protein argonaute-4"
}